{
  "gene_symbol": "CREB3L4",
  "gene_name": "Cyclic AMP-responsive element-binding protein 3-like protein 4",
  "gene": "UniProtKB:Q8TEY5",
  "term_id": "GO:0000981",
  "term_label": "DNA-binding transcription factor activity, RNA polymerase II-specific"
}